{
  "term_id": "UNKNOWN:0001",
  "gene_symbol": "PLEKHB2",
  "term_label": "Unknown molecular function",
  "gene": "UniProtKB:Q96CS7",
  "gene_name": "Pleckstrin homology domain-containing family B member 2"
}